lysine biosynthetic process via diaminopimelate and L-2-acetamido-6-oxoheptanedioate [GO:0033360] (biological process) Relationships: is a type of GO:0009089 Sources: GOC:mah, MetaCyc:PWY-2941 Also known as: lysine anabolism via diaminopimelate and L-2-acetamido-6-oxoheptanedioate, lysine biosynthesis via diaminopimelic acid and L-2-acetamido-6-oxoheptanedioate, lysine biosynthetic process via diaminopimelic acid and L-2-acetamido-6-oxoheptanedioate, lysine formation via diaminopimelate and L-2-acetamido-6-oxoheptanedioate, lysine synthesis via diaminopimelate and L-2-acetamido-6-oxoheptanedioate Definition: The chemical reactions and pathways resulting in the formation of lysine, via the intermediates diaminopimelate and L-2-acetamido-6-oxoheptanedioate; in this pathway tetrahydrodipicolinate is converted to meso-diaminopimelate in four enzymatic steps.